{
  "gene_name": "Zinc finger protein 614",
  "gene": "UniProtKB:Q8N883",
  "term_label": "RNA polymerase II transcription regulatory region sequence-specific DNA binding",
  "gene_symbol": "ZNF614",
  "term_id": "GO:0000977"
}